S-succinyltransferase activity [GO:0016751] (molecular function) Relationships: is a type of S-acyltransferase activity [GO:0016417]; is a type of succinyltransferase activity [GO:0016748] Sources: GOC:ai Subtypes: dihydrolipoyllysine-residue succinyltransferase activity [GO:0004149] Definition: Catalysis of the transfer of a succinyl group to a sulfur atom on the acceptor molecule.